gonadotropin-releasing hormone receptor binding [GO:0031530] (molecular function) Also known as: GnRH receptor binding, gonadotrophin-releasing hormone receptor binding Relationships: is a type of peptide hormone receptor binding [GO:0051428] References: PMID:15196882 Sources: GOC:pr Definition: Binding to a receptor for gonadotropin-releasing hormone (GnRH), a peptide hormone that is synthesized and released by the hypothalamus and is responsible for the release of follicle-stimulating hormone (FSH) and luteinizing hormone (LH) from the anterior pituitary.